nucleotide-excision repair, preincision complex stabilization [GO:0006293] (biological process) Relationships: is a type of GO:0031334; is part of nucleotide-excision repair [GO:0006289] References: PMID:10197977 Sources: GOC:elh Definition: The stabilization of the multiprotein complex involved in damage recognition, DNA helix unwinding, and endonucleolytic cleavage at the site of DNA damage as well as the unwound DNA. The stabilization of the protein-DNA complex ensures proper positioning of the preincision complex before the phosphodiester backbone of the damaged strand is cleaved 3' and 5' of the site of DNA damage.